{
  "term_id": "UNKNOWN:0002",
  "gene_symbol": "TMEM161A",
  "term_label": "Unknown biological process",
  "gene": "UniProtKB:Q9NX61",
  "gene_name": "Transmembrane protein 161A"
}